stereocilium maintenance [GO:0120045] (biological process) References: PMID:27693694 Sources: GOC:krc Relationships: is a type of cellular component maintenance [GO:0043954]; is a type of GO:0060122 Definition: The organization process that preserves a stereocilium in a stable functional or structural state.